{
  "term_label": "potassium channel regulator activity",
  "term_id": "GO:0015459",
  "gene_symbol": "KCNG1",
  "gene_name": "Potassium voltage-gated channel subfamily G member 1",
  "gene": "UniProtKB:Q9UIX4"
}